{
  "gene_name": "Zinc finger protein 70",
  "gene_symbol": "ZNF70",
  "gene": "UniProtKB:Q9UC06",
  "term_id": "GO:0006357",
  "term_label": "regulation of transcription by RNA polymerase II"
}